{
  "term_label": "base-excision repair, gap-filling",
  "gene_name": "DNA polymerase epsilon catalytic subunit A",
  "gene": "UniProtKB:Q07864",
  "term_id": "GO:0006287",
  "gene_symbol": "POLE"
}